{
  "gene_name": "Appetite-regulating hormone",
  "gene": "UniProtKB:Q9UBU3",
  "term_label": "gastric acid secretion",
  "gene_symbol": "GHRL",
  "term_id": "GO:0001696"
}